{
  "gene_symbol": "ADIPOR2",
  "term_id": "GO:0033211",
  "term_label": "adiponectin-activated signaling pathway",
  "gene_name": "Adiponectin receptor protein 2",
  "gene": "UniProtKB:Q86V24"
}